{
  "term_label": "cytoplasm",
  "gene": "UniProtKB:O95299",
  "gene_name": "NADH dehydrogenase [ubiquinone] 1 alpha subcomplex subunit 10, mitochondrial",
  "term_id": "GO:0005737",
  "gene_symbol": "NDUFA10"
}